{
  "term_label": "hydrolase activity, acting on ester bonds",
  "gene_symbol": "C11orf54",
  "gene": "UniProtKB:Q9H0W9",
  "gene_name": "Ester hydrolase C11orf54",
  "term_id": "GO:0016788"
}